3-aci-nitropropanoate oxidase activity [GO:0047557] (MF) Sources: EC:1.7.3.5, RHEA:22372 Also known as: 3-aci-nitropropanoate:oxygen oxidoreductase activity, propionate-3-nitronate oxidase activity Relationships: is a type of GO:0016663 Definition: Catalysis of the reaction: 3-aci-nitropropanoate + H2O + O2 = 3-oxopropanoate + H2O2 + nitrite.